purine-nucleoside phosphorylase activity [GO:0004731] (molecular function) Relationships: is a type of pentosyltransferase activity [GO:0016763] Subtypes: S-methyl-5-thioadenosine phosphorylase activity [GO:0017061] Sources: EC:2.4.2.1 Also known as: inosine phosphorylase activity, PNPase activity, PUNPI, PUNPII, inosine-guanosine phosphorylase activity, purine deoxynucleoside phosphorylase activity, purine deoxyribonucleoside phosphorylase activity, purine nucleoside phosphorylase activity, purine ribonucleoside phosphorylase activity, purine-nucleoside:phosphate ribosyltransferase activity Definition: Catalysis of the reaction: purine nucleoside + phosphate = purine + alpha-D-ribose 1-phosphate.